{
  "gene_symbol": "POMP",
  "gene": "UniProtKB:Q9Y244",
  "gene_name": "Proteasome maturation protein",
  "term_id": "GO:0005737",
  "term_label": "cytoplasm"
}